{
  "term_label": "transcription coactivator activity",
  "gene_name": "Peroxisome proliferator-activated receptor gamma coactivator 1-beta",
  "gene": "UniProtKB:Q86YN6",
  "gene_symbol": "PPARGC1B",
  "term_id": "GO:0003713"
}